{
  "term_label": "canonical Wnt signaling pathway",
  "gene": "UniProtKB:O14641",
  "gene_name": "Segment polarity protein dishevelled homolog DVL-2",
  "gene_symbol": "DVL2",
  "term_id": "GO:0060070"
}